{
  "gene_name": "Selenoprotein H",
  "gene_symbol": "SELENOH",
  "gene": "UniProtKB:Q8IZQ5",
  "term_label": "Golgi apparatus",
  "term_id": "GO:0005794"
}